{
  "gene": "UniProtKB:Q99497",
  "term_id": "GO:0005634",
  "gene_symbol": "PARK7",
  "gene_name": "Parkinson disease protein 7",
  "term_label": "nucleus"
}